extracellular exosome macropinocytosis [GO:0061707] (biological process) Relationships: is a type of macropinocytosis [GO:0044351]; is a type of GO:0051650 References: PMID:24951588 Sources: GOC:dph Definition: The single-organism macropinocytosis process that results in the uptake of an extracellular exosome.